{
  "gene_symbol": "CNTNAP4",
  "term_id": "GO:0005886",
  "term_label": "plasma membrane",
  "gene": "UniProtKB:Q9C0A0",
  "gene_name": "Contactin-associated protein-like 4"
}